MADS box domain binding [GO:0097162] (molecular function) Definition: Binding to a MADS box domain, a protein domain that encodes the DNA-binding MADS domain. The MADS domain binds to DNA sequences of high similarity to the motif CC[A/T]6GG termed the CArG-box. MADS-domain proteins are generally transcription factors. The length of the MADS-box is in the range of 168 to 180 base pairs. References: PMID:18296735 Sources: GOC:yaf, InterPro:IPR002100, Wikipedia:MADS-box Relationships: is a type of protein domain specific binding [GO:0019904]